{
  "gene_name": "Visual system homeobox 1",
  "gene": "UniProtKB:Q9NZR4",
  "gene_symbol": "VSX1",
  "term_label": "neuron development",
  "term_id": "GO:0048666"
}